{
  "gene": "UniProtKB:O60330",
  "term_label": "cell adhesion",
  "gene_name": "Protocadherin gamma-A12",
  "gene_symbol": "PCDHGA12",
  "term_id": "GO:0007155"
}